{
  "term_label": "Unknown cellular component",
  "gene_name": "Fer3-like protein",
  "gene": "UniProtKB:Q96RJ6",
  "gene_symbol": "FERD3L",
  "term_id": "UNKNOWN:0003"
}